{
  "gene_name": "Probable phospholipid-transporting ATPase IIA",
  "term_label": "phospholipid translocation",
  "gene_symbol": "ATP9A",
  "term_id": "GO:0045332",
  "gene": "UniProtKB:O75110"
}